{
  "gene_name": "Eukaryotic translation initiation factor 3 subunit J",
  "gene": "UniProtKB:O75822",
  "gene_symbol": "EIF3J",
  "term_id": "UNKNOWN:0001",
  "term_label": "Unknown molecular function"
}